{
  "gene": "UniProtKB:P51677",
  "term_id": "GO:0019957",
  "gene_symbol": "CCR3",
  "term_label": "C-C chemokine binding",
  "gene_name": "C-C chemokine receptor type 3"
}